regulation of poly(3-hydroxyalkanoate) biosynthetic process [GO:0043286] (biological process) Relationships: is a type of GO:0009889; regulates poly(3-hydroxyalkanoate) biosynthetic process [GO:0042621] Definition: Any process that modulates the frequency, rate or extent of the chemical reactions and pathways resulting in the formation of poly(3-hydroxyalkanoates), polyesters of 3-hydroxyacids produced as intracellular granules by a large variety of bacteria. Sources: GOC:jl Also known as: regulation of PHA, regulation of poly(3-hydroxyalkanoate) anabolism, regulation of poly(3-hydroxyalkanoate) biosynthesis, regulation of poly(3-hydroxyalkanoate) formation, regulation of poly(3-hydroxyalkanoate) synthesis